{
  "gene": "UniProtKB:Q16836",
  "gene_symbol": "HADH",
  "term_id": "GO:0005739",
  "gene_name": "Hydroxyacyl-coenzyme A dehydrogenase, mitochondrial",
  "term_label": "mitochondrion"
}